specification of proximal tubule identity [GO:0072082] (biological process) Sources: GOC:bf, GOC:mtg_kidney_jan10 Subtypes: specification of pronephric proximal tubule identity [GO:0039004], specification of mesonephric proximal tubule identity [GO:0061284], specification of metanephric proximal tubule identity [GO:0072297] Relationships: is a type of specification of nephron tubule identity [GO:0072081]; is part of proximal tubule morphogenesis [GO:0072158] Definition: The process in which the proximal tubule of the kidney nephron acquires its identity.